{
  "term_id": "UNKNOWN:0003",
  "gene_name": "Endogenous retrovirus group FC1 member 1 Env polyprotein",
  "term_label": "Unknown cellular component",
  "gene_symbol": "ERVFC1-1",
  "gene": "UniProtKB:P60608"
}